positive regulation of basidium development [GO:0075315] (BP) Sources: GOC:pamgo_curators Definition: Any process that activates, maintains or increases the frequency, rate or extent of basidium development, a process that leads to the formation of basidium, a small, specialized club-shaped structure typically bearing four basidiospores at the tips of minute projections. The basidium is unique to basidiomycetes and distinguishes them from other kinds of fungi. Relationships: is a type of positive regulation of spore-bearing organ development [GO:0075261]; is a type of regulation of basidium development [GO:0075314]; positively regulates basidium development [GO:0075313]